aminoglycoside 2''-nucleotidyltransferase activity [GO:0008871] (molecular function) Also known as: NTP:gentamicin 2''-nucleotidyltransferase activity, gentamicin 2''- adenylyltransferase activity, gentamicin 2''-nucleotidyltransferase activity, gentamycin 2''-nucleotidyltransferase activity, 2''-aminoglycoside nucleotidyltransferase activity Sources: EC:2.7.7.46, GOC:cb Definition: Catalysis of the reaction: nucleoside triphosphate + aminoglycoside = diphosphate + 2''-nucleotidylaminoglycoside. Relationships: is_a aminoglycoside nucleotidyltransferase activity [GO:0034068]